{
  "gene": "UniProtKB:Q9Y484",
  "term_label": "nucleophagy",
  "gene_symbol": "WDR45",
  "gene_name": "WD repeat domain phosphoinositide-interacting protein 4",
  "term_id": "GO:0044804"
}